{
  "term_id": "UNKNOWN:0001",
  "gene": "UniProtKB:Q96FF7",
  "gene_symbol": "MISP3",
  "gene_name": "Uncharacterized protein MISP3",
  "term_label": "Unknown molecular function"
}